{
  "term_label": "cell projection",
  "gene_name": "Glial fibrillary acidic protein",
  "gene": "UniProtKB:P14136",
  "gene_symbol": "GFAP",
  "term_id": "GO:0042995"
}